modification-dependent protein binding [GO:0140030] (molecular function) Relationships: is a type of protein binding [GO:0005515] Also known as: modified protein binding Subtypes: polyubiquitin modification-dependent protein binding [GO:0031593], phosphorylation-dependent protein binding [GO:0140031], glycosylation-dependent protein binding [GO:0140032], GO:0140033, methylation-dependent protein binding [GO:0140034], GO:0160002 Note: This term should only be used when the binding is shown to require a post-translational modification: the interaction needs to be tested with and without the PTM. The binding does not need to be at the site of the modification. It may be that the PTM causes a conformational change that allows binding of the protein to another region; this type of modification-dependent protein binding is valid for annotation to this term. Definition: Binding to a protein upon post-translation modification of the target protein. References: PMID:26060076